positive regulation of cardiocyte differentiation [GO:1905209] (biological process) References: PMID:23069713 Sources: GOC:BHF, GOC:BHF_miRNA, GOC:TermGenie, GOC:bc, GO_REF:0000058 Definition: Any process that activates or increases the frequency, rate or extent of cardiocyte differentiation. Also known as: positive regulation of cardiac cell differentiation, positive regulation of heart cell differentiation, up regulation of cardiac cell differentiation, up regulation of cardiocyte differentiation, up regulation of heart cell differentiation, up-regulation of cardiac cell differentiation, up-regulation of cardiocyte differentiation, up-regulation of heart cell differentiation, upregulation of cardiac cell differentiation, upregulation of cardiocyte differentiation, upregulation of heart cell differentiation, activation of cardiac cell differentiation, activation of cardiocyte differentiation, activation of heart cell differentiation Relationships: is a type of positive regulation of cell differentiation [GO:0045597]; is a type of positive regulation of multicellular organismal process [GO:0051240]; is a type of regulation of cardiocyte differentiation [GO:1905207]; positively regulates cardiocyte differentiation [GO:0035051] Subtypes: positive regulation of cardioblast differentiation [GO:0051891], positive regulation of endocardial cushion cell differentiation [GO:0120075], GO:2000724, positive regulation of cardiac muscle cell differentiation [GO:2000727]